{
  "gene_symbol": "C8orf74",
  "term_id": "UNKNOWN:0002",
  "gene_name": "Uncharacterized protein C8orf74",
  "term_label": "Unknown biological process",
  "gene": "UniProtKB:Q6P047"
}